seed germination on parent plant [GO:0048623] (biological process) Sources: GOC:go_curators Relationships: is_a seed germination [GO:0009845] Definition: The process in which a seed germinates before being shed from the parent plant. Also known as: non-vegetative vivipary, vivipary, pre-harvest sprouting